{
  "term_label": "serine-type endopeptidase activity",
  "gene_name": "Chymase",
  "gene": "UniProtKB:P23946",
  "term_id": "GO:0004252",
  "gene_symbol": "CMA1"
}